{
  "term_label": "endoplasmic reticulum-Golgi intermediate compartment",
  "term_id": "GO:0005793",
  "gene_symbol": "MGAT4A",
  "gene": "UniProtKB:Q9UM21",
  "gene_name": "Alpha-1,3-mannosyl-glycoprotein 4-beta-N-acetylglucosaminyltransferase A"
}